{
  "gene": "UniProtKB:Q9Y6G9",
  "term_id": "GO:0045504",
  "term_label": "dynein heavy chain binding",
  "gene_name": "Cytoplasmic dynein 1 light intermediate chain 1",
  "gene_symbol": "DYNC1LI1"
}